{
  "gene_symbol": "CACNG5",
  "term_id": "GO:0098970",
  "gene_name": "Voltage-dependent calcium channel gamma-5 subunit",
  "gene": "UniProtKB:Q9UF02",
  "term_label": "postsynaptic neurotransmitter receptor diffusion trapping"
}